{
  "gene": "UniProtKB:Q8N9E0",
  "term_id": "UNKNOWN:0003",
  "gene_symbol": "FAM133A",
  "gene_name": "Protein FAM133A",
  "term_label": "Unknown cellular component"
}